Lewy neurite [GO:0097462] (CC) Sources: NIF_Subcellular:sao601362597 Definition: Elongated neuronal process, often with side branches and more than one branching point, described in brains of patients with Parkinson's disease. Lewy neurites stain positively for ubiquitin in brainstem and forebrain regions affected in Parkinson's disease. Relationships: is a type of neuron projection [GO:0043005]